regulation of endothelial cell chemotaxis [GO:2001026] (BP) Definition: Any process that modulates the frequency, rate or extent of endothelial cell chemotaxis. Sources: GOC:BHF Relationships: is a type of GO:0010594; is a type of regulation of chemotaxis [GO:0050920]; regulates endothelial cell chemotaxis [GO:0035767] Subtypes: regulation of endothelial cell chemotaxis to fibroblast growth factor [GO:2000544], negative regulation of endothelial cell chemotaxis [GO:2001027], positive regulation of endothelial cell chemotaxis [GO:2001028]